interleukin-27-mediated signaling pathway [GO:0070106] (biological process) Relationships: is a type of cytokine-mediated signaling pathway [GO:0019221] Sources: GOC:BHF, GOC:add, GOC:mah, GOC:signaling Also known as: IL-27-mediated signaling pathway, IL27RA/IL6ST signaling pathway, interleukin-27-mediated signalling pathway Regulation: regulated by GO:0070107; RO_0002212 by negative regulation of interleukin-27-mediated signaling pathway [GO:0070108]; positively regulated by positive regulation of interleukin-27-mediated signaling pathway [GO:0070109] Definition: The series of molecular signals initiated by interleukin-27 binding to a receptor on the surface of a target cell, and ending with the regulation of a downstream cellular process, e.g. transcription.